{
  "gene_symbol": "KIAA0825",
  "term_label": "Unknown cellular component",
  "term_id": "UNKNOWN:0003",
  "gene_name": "Uncharacterized protein KIAA0825",
  "gene": "UniProtKB:Q8IV33"
}